{
  "term_label": "N-acetylmuramoyl-L-alanine amidase activity",
  "gene": "UniProtKB:O75594",
  "gene_name": "Peptidoglycan recognition protein 1",
  "gene_symbol": "PGLYRP1",
  "term_id": "GO:0008745"
}